{
  "gene_symbol": "SLC35C1",
  "gene": "UniProtKB:Q96A29",
  "gene_name": "GDP-fucose transporter 1",
  "term_label": "antiporter activity",
  "term_id": "GO:0015297"
}